{
  "term_label": "regulation of transcription by RNA polymerase II",
  "gene_name": "Zinc finger protein 577",
  "term_id": "GO:0006357",
  "gene": "UniProtKB:Q9BSK1",
  "gene_symbol": "ZNF577"
}